{
  "term_id": "GO:0000978",
  "gene_symbol": "NFIB",
  "gene": "UniProtKB:O00712",
  "term_label": "RNA polymerase II cis-regulatory region sequence-specific DNA binding",
  "gene_name": "Nuclear factor 1 B-type"
}